{
  "term_id": "GO:0030178",
  "term_label": "negative regulation of Wnt signaling pathway",
  "gene_name": "Sclerostin domain-containing protein 1",
  "gene": "UniProtKB:Q6X4U4",
  "gene_symbol": "SOSTDC1"
}